{
  "gene_name": "Rab-like protein 2A",
  "term_id": "GO:0006886",
  "term_label": "intracellular protein transport",
  "gene": "UniProtKB:Q9UBK7",
  "gene_symbol": "RABL2A"
}